response to osmotic stress [GO:0006970] (biological process) Definition: Any process that results in a change in state or activity of a cell or an organism (in terms of movement, secretion, enzyme production, gene expression, etc.) as a result of a stimulus indicating an increase or decrease in the concentration of solutes outside the organism or cell. Relationships: is a type of response to stress [GO:0006950]; is a type of response to abiotic stimulus [GO:0009628] Sources: GOC:jl Subtypes: GO:0006971, hyperosmotic response [GO:0006972], GO:0009651, response to non-ionic osmotic stress [GO:0010335], GO:0043575, cellular response to osmotic stress [GO:0071470] Regulation: regulated by GO:0047484 Also known as: osmotic response, osmotic stress response